{
  "term_label": "cytoplasm",
  "gene": "UniProtKB:O15013",
  "gene_symbol": "ARHGEF10",
  "term_id": "GO:0005737",
  "gene_name": "Rho guanine nucleotide exchange factor 10"
}